piRNA-mediated gene silencing by mRNA destabilization [GO:0140991] (biological process) Subtypes: GO:0141009 Definition: A cytoplasmic post-transcriptional gene silencing pathway in which piRNAs direct the cleavage of target mRNAs. The target mRNA, often transcribed from a transposable element, is destabilized by the activity of a PIWI class endonuclease within the piRNA-induced silencing complex. This may also be accompanied by mRNA deadenylation and decapping. References: PMID:29281264, PMID:33419460 Relationships: is a type of regulatory ncRNA-mediated post-transcriptional gene silencing [GO:0035194]; is a type of mRNA destabilization [GO:0061157]